{
  "gene_name": "Immunoglobulin heavy variable 5-10-1",
  "gene": "UniProtKB:A0A0J9YXX1",
  "term_id": "GO:0003823",
  "gene_symbol": "IGHV5-10-1",
  "term_label": "antigen binding"
}